{
  "term_label": "lipid droplet",
  "gene": "UniProtKB:Q7Z5P4",
  "gene_symbol": "HSD17B13",
  "gene_name": "17-beta-hydroxysteroid dehydrogenase 13",
  "term_id": "GO:0005811"
}